TRAIL death-inducing signaling complex assembly [GO:1903074] (biological process) Relationships: is_a death-inducing signaling complex assembly [GO:0071550]; is part of TRAIL-activated apoptotic signaling pathway [GO:0036462] Definition: The aggregation, arrangement and bonding together of a set of components to form a TRAIL death-inducing signaling complex. Also known as: TRAIL DISC assembly, TRAIL DISC formation, TRAIL death-inducing signaling complex formation, TRAIL death-inducing signalling complex assembly, TRAIL death-inducing signalling complex formation References: PMID:21785459 Sources: GOC:PARL, GOC:TermGenie, GOC:bf, GO_REF:0000079